{
  "gene": "UniProtKB:P0C5Y4",
  "term_label": "Unknown molecular function",
  "term_id": "UNKNOWN:0001",
  "gene_name": "Keratin-associated protein 1-4",
  "gene_symbol": "KRTAP1-4"
}